{
  "gene_symbol": "CEP20",
  "gene": "UniProtKB:Q96NB1",
  "term_id": "GO:0005813",
  "gene_name": "Centrosomal protein 20",
  "term_label": "centrosome"
}